inflammatory cell apoptotic process [GO:0006925] (biological process) Definition: Any apoptotic process in an inflammatory cell, any cell participating in the inflammatory response to a foreign substance e.g. neutrophil, macrophage. Sources: GOC:jl, GOC:mtg_apoptosis Subtypes: neutrophil apoptotic process [GO:0001781], GO:0071888 Relationships: is a type of GO:0006915 Also known as: apoptosis of inflammatory cells, inflammatory cell programmed cell death by apoptosis, killing of inflammatory cells, programmed cell death of inflammatory cells by apoptosis, programmed cell death, inflammatory cells, inflammatory cell apoptosis